morphogen activity [GO:0016015] (molecular function) Definition: Acts as a trigger for a pattern specification process when present at a specific concentration within a gradient. Relationships: is a type of receptor ligand activity [GO:0048018] Sources: GOC:go_curators